{
  "gene_symbol": "GNRH2",
  "term_id": "UNKNOWN:0002",
  "gene": "UniProtKB:O43555",
  "gene_name": "Progonadoliberin-2",
  "term_label": "Unknown biological process"
}